{
  "term_label": "Unknown biological process",
  "gene": "UniProtKB:P51814",
  "gene_symbol": "ZNF41",
  "gene_name": "Zinc finger protein 41",
  "term_id": "UNKNOWN:0002"
}